{
  "gene_symbol": "SYT13",
  "term_id": "GO:0005544",
  "gene_name": "Synaptotagmin-13",
  "term_label": "calcium-dependent phospholipid binding",
  "gene": "UniProtKB:Q7L8C5"
}